bone mineralization involved in bone maturation [GO:0035630] (biological process) Relationships: is a type of bone mineralization [GO:0030282]; is part of ossification involved in bone maturation [GO:0043931] Sources: GOC:BHF, GOC:bf Note: Bone mineralization can also occur after a fracture and as a response to stress; in these cases, consider using the term 'bone mineralization ; GO:0030282'. Definition: The deposition of hydroxyapatite, involved in the progression of the skeleton from its formation to its mature state. Regulation: regulated by regulation of bone mineralization involved in bone maturation [GO:1900157]; negatively regulated by negative regulation of bone mineralization involved in bone maturation [GO:1900158]; positively regulated by positive regulation of bone mineralization involved in bone maturation [GO:1900159]